{
  "term_id": "GO:0003779",
  "gene": "UniProtKB:O43312",
  "gene_symbol": "MTSS1",
  "gene_name": "Protein MTSS 1",
  "term_label": "actin binding"
}